{
  "gene_name": "5-hydroxytryptamine receptor 1D",
  "term_id": "GO:0005886",
  "gene_symbol": "HTR1D",
  "term_label": "plasma membrane",
  "gene": "UniProtKB:P28221"
}